{
  "term_label": "nucleoplasm",
  "gene_name": "Poly(rC)-binding protein 1",
  "gene": "UniProtKB:Q15365",
  "gene_symbol": "PCBP1",
  "term_id": "GO:0005654"
}